{
  "term_label": "Unknown biological process",
  "gene_symbol": "PRR23A",
  "gene_name": "Proline-rich protein 23A",
  "term_id": "UNKNOWN:0002",
  "gene": "UniProtKB:A6NEV1"
}